leukocyte migration involved in immune response [GO:0002522] (biological process) Definition: The movement of a leukocyte within or between different tissues and organs of the body as part of an immune response. References: PMID:14680625, PMID:14708592, PMID:7507411, PMID:8600538 Sources: GOC:add, ISBN:0781735149 Also known as: immune cell migration during immune response, immune cell trafficking during immune response, leucocyte migration during immune response, leucocyte trafficking during immune response, leukocyte trafficking during immune response Relationships: is a type of immune effector process [GO:0002252]; is_a GO:0050900; is part of GO:0006955 Subtypes: leukocyte chemotaxis involved in immune response [GO:0002233]